{
  "gene": "UniProtKB:A6NGH7",
  "gene_symbol": "CCDC160",
  "term_id": "UNKNOWN:0002",
  "gene_name": "Coiled-coil domain-containing protein 160",
  "term_label": "Unknown biological process"
}